{
  "gene_name": "Calpain-2 catalytic subunit",
  "term_id": "GO:0004198",
  "gene": "UniProtKB:P17655",
  "term_label": "calcium-dependent cysteine-type endopeptidase activity",
  "gene_symbol": "CAPN2"
}